immune response-regulating cell surface receptor signaling pathway [GO:0002768] (biological process) Subtypes: immune response-activating cell surface receptor signaling pathway [GO:0002429], immune response-regulating cell surface receptor signaling pathway involved in phagocytosis [GO:0002433], immune response-inhibiting cell surface receptor signaling pathway [GO:0002767], Fc receptor signaling pathway [GO:0038093] Relationships: is a type of immune response-regulating signaling pathway [GO:0002764]; is_a cell surface receptor signaling pathway [GO:0007166] Also known as: immune response-regulating cell surface receptor signalling pathway Definition: The series of molecular signals initiated by an extracellular ligand binding to a receptor on the surface of the target cell capable of activating, perpetuating, or inhibiting an immune response. References: PMID:15771571 Sources: GOC:add, ISBN:0781735149